{
  "term_id": "GO:0004984",
  "gene": "UniProtKB:Q8NGK1",
  "term_label": "olfactory receptor activity",
  "gene_symbol": "OR51G1",
  "gene_name": "Olfactory receptor 51G1"
}